{
  "gene_symbol": "SEMA4D",
  "gene": "UniProtKB:Q92854",
  "term_label": "extracellular space",
  "term_id": "GO:0005615",
  "gene_name": "Semaphorin-4D"
}